{
  "term_label": "adherens junction",
  "gene_name": "LIM domain-containing protein 1",
  "gene_symbol": "LIMD1",
  "term_id": "GO:0005912",
  "gene": "UniProtKB:Q9UGP4"
}